{
  "term_id": "GO:0016323",
  "gene": "UniProtKB:P11166",
  "term_label": "basolateral plasma membrane",
  "gene_name": "Solute carrier family 2, facilitated glucose transporter member 1",
  "gene_symbol": "SLC2A1"
}